positive regulation of interleukin-27 production [GO:0032751] (biological process) Also known as: positive regulation of IL-27 production, up regulation of interleukin-27 production, up-regulation of interleukin-27 production, upregulation of interleukin-27 production, activation of interleukin-27 production, positive regulation of interleukin-27 anabolism, positive regulation of interleukin-27 biosynthetic process, stimulation of interleukin-27 production Definition: Any process that activates or increases the frequency, rate, or extent of interleukin-27 production. Relationships: is a type of positive regulation of cytokine production [GO:0001819]; is a type of GO:0032671; positively regulates GO:0032631 Sources: GOC:mah